{
  "gene_symbol": "GUCY2F",
  "gene_name": "Retinal guanylyl cyclase 2",
  "term_label": "cGMP biosynthetic process",
  "term_id": "GO:0006182",
  "gene": "UniProtKB:P51841"
}